{
  "term_id": "GO:0000981",
  "gene_name": "Transcription factor ATOH1",
  "gene": "UniProtKB:Q92858",
  "term_label": "DNA-binding transcription factor activity, RNA polymerase II-specific",
  "gene_symbol": "ATOH1"
}